negative regulation of mitotic cell cycle [GO:0045930] (biological process) Definition: Any process that stops, prevents or reduces the rate or extent of progression through the mitotic cell cycle. Relationships: is a type of regulation of mitotic cell cycle [GO:0007346]; is a type of GO:0045786; negatively regulates mitotic cell cycle [GO:0000278] Subtypes: mitotic cell cycle G1 arrest in response to pheromone [GO:0000751], GO:0007093, negative regulation of mitotic nuclear division [GO:0045839], negative regulation of mitotic cell cycle, embryonic [GO:0045976], cell cycle switching, mitotic to meiotic cell cycle [GO:0051728], negative regulation of mitotic cell cycle phase transition [GO:1901991], GO:1903464 Also known as: down regulation of progression through mitotic cell cycle, down-regulation of progression through mitotic cell cycle, downregulation of progression through mitotic cell cycle, negative regulation of mitotic cell cycle progression, negative regulation of progression through mitotic cell cycle, inhibition of progression through mitotic cell cycle Sources: GOC:dph, GOC:go_curators, GOC:tb